{
  "gene_name": "Sodium channel subunit beta-1",
  "gene_symbol": "SCN1B",
  "term_label": "sodium ion transmembrane transport",
  "gene": "UniProtKB:Q07699",
  "term_id": "GO:0035725"
}